{
  "gene_name": "Growth_differentiation factor 3",
  "gene": "UniProtKB:Q9NR23",
  "gene_symbol": "GDF3",
  "term_id": "GO:0005615",
  "term_label": "extracellular space"
}